{
  "gene_symbol": "GPM6A",
  "term_label": "neuronal cell body",
  "gene": "UniProtKB:P51674",
  "term_id": "GO:0043025",
  "gene_name": "Neuronal membrane glycoprotein M6-a"
}